{
  "term_id": "GO:0004984",
  "term_label": "olfactory receptor activity",
  "gene_symbol": "OR56A1",
  "gene": "UniProtKB:Q8NGH5",
  "gene_name": "Olfactory receptor 56A1"
}